{
  "gene_name": "Adiponectin receptor protein 1",
  "term_label": "adiponectin-activated signaling pathway",
  "gene_symbol": "ADIPOR1",
  "term_id": "GO:0033211",
  "gene": "UniProtKB:Q96A54"
}